{
  "term_label": "protein-membrane adaptor activity",
  "gene": "UniProtKB:Q9UH99",
  "term_id": "GO:0043495",
  "gene_symbol": "SUN2",
  "gene_name": "SUN domain-containing protein 2"
}